{
  "term_id": "UNKNOWN:0003",
  "gene_symbol": "SPATA31A1",
  "term_label": "Unknown cellular component",
  "gene_name": "Spermatogenesis-associated protein 31A1",
  "gene": "UniProtKB:Q5TZJ5"
}